{
  "gene": "UniProtKB:P00558",
  "gene_name": "Phosphoglycerate kinase 1",
  "term_label": "gluconeogenesis",
  "gene_symbol": "PGK1",
  "term_id": "GO:0006094"
}